negative regulation of telomerase RNA localization to Cajal body [GO:1904873] (biological process) References: PMID:25467444 Sources: GOC:BHF, GOC:BHF_telomere, GOC:TermGenie, GOC:nc, GO_REF:0000058 Relationships: is a type of negative regulation of biological process [GO:0048519]; is_a regulation of telomerase RNA localization to Cajal body [GO:1904872]; negatively regulates GO:0090671 Also known as: down regulation of telomerase RNA localization to Cajal body, down-regulation of telomerase RNA localization to Cajal body, downregulation of telomerase RNA localization to Cajal body, inhibition of telomerase RNA localization to Cajal body Definition: Any process that stops, prevents or reduces the frequency, rate or extent of telomerase RNA localization to Cajal body.